negative regulation of superoxide anion generation [GO:0032929] (biological process) Relationships: is a type of regulation of superoxide anion generation [GO:0032928]; is a type of negative regulation of reactive oxygen species metabolic process [GO:2000378]; negatively regulates superoxide anion generation [GO:0042554] Also known as: down regulation of superoxide release, down-regulation of superoxide release, downregulation of superoxide release, negative regulation of superoxide release, inhibition of superoxide release Definition: Any process that stops, prevents, or reduces the frequency, rate or extent of enzymatic generation of superoxide by a cell. Sources: GOC:mah